{
  "gene_name": "Uncharacterized protein (Fragment)",
  "gene": "UniProtKB:A0A087WWU0",
  "term_id": "UNKNOWN:0003",
  "term_label": "Unknown cellular component",
  "gene_symbol": "A0A087WWU0"
}